T=16 icosahedral viral capsid [GO:0039622] (cellular component) Definition: The protein coat that surrounds the infective nucleic acid in some virus particles where the subunits (capsomeres) are arranged to form an icosahedron with T=16 symmetry. The T=16 capsid is composed of 12 pentameric and 150 hexameric capsomeres. Relationships: is a type of GO:0019030 Sources: VZ:807